oxaloacetate transport [GO:0015729] (biological process) Subtypes: oxaloacetate(2-) transmembrane transport [GO:1902356] Relationships: is a type of GO:0015740 Sources: GOC:krc Definition: The directed movement of oxaloacetate, the anion of oxobutanedioic acid, into, out of or within a cell, or between cells, by means of some agent such as a transporter or pore.